{
  "term_id": "GO:0042073",
  "gene": "UniProtKB:P20794",
  "gene_symbol": "MAK",
  "term_label": "intraciliary transport",
  "gene_name": "Serine_threonine-protein kinase MAK"
}